{
  "term_label": "endosome",
  "gene": "UniProtKB:Q9H201",
  "gene_name": "Epsin-3",
  "gene_symbol": "EPN3",
  "term_id": "GO:0005768"
}